RAD52-ERCC4-ERCC1 complex [GO:0070312] (cellular component) Definition: A nucleotide-excision repair complex formed by the association of the heterodimeric endonuclease XPF/ERCC4-ERCC1 (Rad1p and Rad10p in S. cerevisiae) with the RAD52 protein. References: PMID:14734547 Note: Note that process and function information are included in the term and definition for the purpose of describing and distinguishing the complex. Relationships: is a type of nucleotide-excision repair complex [GO:0000109]